phosphoenolpyruvate transmembrane transport [GO:0089722] (biological process) Sources: GOC:dos Subtypes: phosphoenolpyruvate transmembrane import into Golgi lumen [GO:1990536] Relationships: is a type of GO:0015714; is a type of carboxylic acid transmembrane transport [GO:1905039] Definition: The directed movement of phosphoenolpytuvate across a membrane.